{
  "term_id": "GO:0016887",
  "gene_name": "Chromodomain-helicase-DNA-binding protein 7",
  "gene_symbol": "CHD7",
  "gene": "UniProtKB:Q9P2D1",
  "term_label": "ATP hydrolysis activity"
}